{
  "gene_name": "Endoplasmic reticulum membrane sensor NFE2L1",
  "term_id": "GO:0005634",
  "gene_symbol": "NFE2L1",
  "gene": "UniProtKB:Q14494",
  "term_label": "nucleus"
}